tungstate ion transport [GO:0070614] (biological process) Sources: GOC:dh Relationships: is a type of inorganic anion transport [GO:0015698] Definition: The directed movement of tungstate (WO4 2-) ions into, out of or within a cell, or between cells, by means of some agent such as a transporter or pore. Tungstate is a bivalent oxoanion of tungsten.